{
  "gene_name": "Homeobox protein Nkx-3.1",
  "term_label": "regulation of transcription by RNA polymerase II",
  "gene": "UniProtKB:Q99801",
  "gene_symbol": "NKX3-1",
  "term_id": "GO:0006357"
}